GATA2-TAL1-TCF3-Lmo2 complex [GO:0070354] (cellular component) References: PMID:7568177 Relationships: is a type of nuclear protein-containing complex [GO:0140513] Definition: A protein complex that contains the zinc finger transcription factor GATA2, the LIM domain protein Lmo2 (RBTN2), the basic helix-loop-helix protein TAL1 and its binding partner TCF3. The complex is involved transcriptional regulation in hematopoiesis.